{
  "term_id": "GO:0000398",
  "term_label": "mRNA splicing, via spliceosome",
  "gene_name": "Putative small nuclear ribonucleoprotein G-like protein 15",
  "gene": "UniProtKB:A8MWD9",
  "gene_symbol": "SNRPGP15"
}